{
  "gene": "UniProtKB:O00562",
  "gene_symbol": "PITPNM1",
  "gene_name": "Membrane-associated phosphatidylinositol transfer protein 1",
  "term_label": "cytoplasm",
  "term_id": "GO:0005737"
}